{
  "gene_symbol": "ITGBL1",
  "gene": "UniProtKB:O95965",
  "term_label": "cell migration",
  "gene_name": "Integrin beta-like protein 1",
  "term_id": "GO:0016477"
}